{
  "gene_name": "Olfactory receptor 2T1",
  "gene_symbol": "OR2T1",
  "term_id": "GO:0004984",
  "term_label": "olfactory receptor activity",
  "gene": "UniProtKB:O43869"
}